peptidyl-proline 4-dioxygenase binding [GO:0098650] (molecular function) Relationships: is a type of enzyme binding [GO:0019899] Sources: GOC:dos, GOC:kvm Definition: Binding to a peptidyl-proline 4-dioxygenase.